{
  "term_id": "GO:0005882",
  "gene_symbol": "PPL",
  "gene": "UniProtKB:O60437",
  "gene_name": "Periplakin",
  "term_label": "intermediate filament"
}